{
  "gene_name": "Uncharacterized protein",
  "gene_symbol": "LOC101059915",
  "gene": "UniProtKB:A0A1B0GWI6",
  "term_label": "Unknown cellular component",
  "term_id": "UNKNOWN:0003"
}